somatic diversification of immune receptors via alternate splicing [GO:0002563] (biological process) References: PMID:16166509 Sources: GOC:add, ISBN:0781735149 Relationships: is a type of somatic diversification of immune receptors [GO:0002200] Definition: The process in which immune receptor genes are diversified through alternate splicing. Subtypes: alternate splicing of immunoglobulin genes [GO:0002564]